{
  "gene_name": "Regulator of nonsense transcripts 2",
  "term_id": "GO:0035145",
  "gene_symbol": "UPF2",
  "term_label": "exon-exon junction complex",
  "gene": "UniProtKB:Q9HAU5"
}